{
  "term_label": "pantetheine-phosphate adenylyltransferase activity",
  "gene_symbol": "COASY",
  "gene_name": "Bifunctional coenzyme A synthase",
  "term_id": "GO:0004595",
  "gene": "UniProtKB:Q13057"
}